{
  "term_id": "GO:0048015",
  "term_label": "phosphatidylinositol-mediated signaling",
  "gene_symbol": "PLCH2",
  "gene_name": "1-phosphatidylinositol 4,5-bisphosphate phosphodiesterase eta-2",
  "gene": "UniProtKB:O75038"
}